{
  "term_label": "plasma membrane",
  "gene_name": "Proton channel OTOP2",
  "gene": "UniProtKB:Q7RTS6",
  "gene_symbol": "OTOP2",
  "term_id": "GO:0005886"
}